regulation of fractalkine production [GO:0032644] (biological process) Definition: Any process that modulates the frequency, rate, or extent of fractalkine production. Subtypes: negative regulation of fractalkine production [GO:0032684], positive regulation of fractalkine production [GO:0032724] Relationships: is a type of regulation of chemokine production [GO:0032642]; regulates fractalkine production [GO:0032603] Also known as: regulation of CX3CL1 biosynthesis, regulation of CX3CL1 production, regulation of fractalkine biosynthetic process Sources: GOC:mah